{
  "gene": "UniProtKB:Q7Z6K4",
  "gene_symbol": "NRARP",
  "term_id": "UNKNOWN:0003",
  "term_label": "Unknown cellular component",
  "gene_name": "Notch-regulated ankyrin repeat-containing protein"
}